{
  "term_label": "cytoplasm",
  "gene_name": "Spermatogenesis-associated protein 2-like protein",
  "gene": "UniProtKB:Q8IUW3",
  "term_id": "GO:0005737",
  "gene_symbol": "SPATA2L"
}